{
  "term_label": "Unknown cellular component",
  "gene": "UniProtKB:A0A1B0GVV1",
  "gene_symbol": "SMIM35",
  "gene_name": "Small integral membrane protein 35",
  "term_id": "UNKNOWN:0003"
}